{
  "gene": "UniProtKB:Q12907",
  "gene_symbol": "LMAN2",
  "gene_name": "Vesicular integral-membrane protein VIP36",
  "term_id": "GO:0005537",
  "term_label": "D-mannose binding"
}